maturation of SSU-rRNA from tricistronic rRNA transcript (SSU-rRNA, 5.8S rRNA, LSU-rRNA) [GO:0000462] (BP) Relationships: is_a maturation of SSU-rRNA [GO:0030490] Definition: Any process involved in the maturation of a precursor Small SubUnit (SSU) ribosomal RNA (rRNA) molecule into a mature SSU-rRNA molecule from the pre-rRNA molecule originally produced as a tricistronic rRNA transcript that contains the Small Subunit (SSU) rRNA, 5.8S rRNA, and the Large Subunit (LSU) in that order from 5' to 3' along the primary transcript. Sources: GOC:curators Also known as: maturation of 18S rRNA